{
  "gene": "UniProtKB:P49247",
  "gene_symbol": "RPIA",
  "term_label": "ribose-5-phosphate isomerase activity",
  "term_id": "GO:0004751",
  "gene_name": "Ribose-5-phosphate isomerase"
}